{
  "term_id": "GO:0008270",
  "gene_name": "Zinc-regulated GTPase metalloprotein activator 1A",
  "term_label": "zinc ion binding",
  "gene_symbol": "ZNG1A",
  "gene": "UniProtKB:Q9BRT8"
}